{
  "term_label": "endoplasmic reticulum",
  "gene_name": "Cartilage-associated protein",
  "gene": "UniProtKB:O75718",
  "gene_symbol": "CRTAP",
  "term_id": "GO:0005783"
}